alkane transport [GO:0015895] (biological process) Relationships: is a type of transport [GO:0006810] Definition: The directed movement of alkanes into, out of or within a cell, or between cells, by means of some agent such as a transporter or pore. Alkanes are saturated aliphatic hydrocarbon compounds. Sources: GOC:ai